detection of mechanical stimulus involved in echolocation [GO:0050972] (biological process) Also known as: echolocation, detection of mechanical stimulus, echolocation, sensory detection of mechanical stimulus, echolocation, sensory transduction of mechanical stimulus, sensory detection of mechanical stimulus during echolocation, sensory transduction of mechanical stimulus during echolocation Relationships: is a type of detection of mechanical stimulus involved in sensory perception [GO:0050974]; is part of GO:0050959 Definition: The series of events involved in echolocation in which a mechanical stimulus is received and converted into a molecular signal. The stimulus is in the form of a reflected sound wave (an echo), which the organism uses to determine the distance to the object that reflected the sound wave. Sources: GOC:ai, GOC:dos